{
  "term_label": "nucleus",
  "term_id": "GO:0005634",
  "gene_name": "MBT domain-containing protein 1",
  "gene": "UniProtKB:Q05BQ5",
  "gene_symbol": "MBTD1"
}